{
  "term_label": "hippo signaling",
  "gene_symbol": "AMOTL2",
  "term_id": "GO:0035329",
  "gene_name": "Angiomotin-like protein 2",
  "gene": "UniProtKB:Q9Y2J4"
}